lipopolysaccharide glucosyltransferase I activity [GO:0008919] (molecular function) Relationships: is a type of UDP-glucosyltransferase activity [GO:0035251]; is part of GO:0009103 Also known as: LPS glucosyltransferase I activity, UDP-glucose:lipopolysaccharide glucosyltransferase activity, UDPglucose:lipopolysaccharide glucosyltransferase I, UDPglucose:lipopolysaccharide glucosyltransferase activity, lipopolysaccharide glucosyltransferase activity, uridine diphosphate glucose:lipopolysaccharide glucosyltransferase I, uridine diphosphoglucose-lipopolysaccharide glucosyltransferase activity Sources: EC:2.4.1.58 Definition: Catalysis of the reaction: UDP-glucose + lipopolysaccharide = UDP + D-glucosyl-lipopolysaccharide.